{
  "term_id": "UNKNOWN:0001",
  "gene_name": "Rho GTPase-activating protein 21",
  "term_label": "Unknown molecular function",
  "gene_symbol": "ARHGAP21",
  "gene": "UniProtKB:Q5T5U3"
}